{
  "gene_name": "Uncharacterized protein",
  "term_label": "Unknown molecular function",
  "gene_symbol": "A0A8V8TPW5",
  "term_id": "UNKNOWN:0001",
  "gene": "UniProtKB:A0A8V8TPW5"
}